{
  "gene": "UniProtKB:Q8TBF8",
  "term_id": "UNKNOWN:0003",
  "gene_name": "Protein FAM81A",
  "term_label": "Unknown cellular component",
  "gene_symbol": "FAM81A"
}